{
  "term_label": "positive regulation of blood pressure",
  "gene": "UniProtKB:P43220",
  "gene_symbol": "GLP1R",
  "gene_name": "Glucagon-like peptide 1 receptor",
  "term_id": "GO:0045777"
}